{
  "term_label": "cytoplasm",
  "gene_name": "Vinculin",
  "term_id": "GO:0005737",
  "gene_symbol": "VCL",
  "gene": "UniProtKB:P18206"
}